{
  "term_id": "UNKNOWN:0002",
  "gene_name": "ATP-dependent RNA helicase DHX29",
  "term_label": "Unknown biological process",
  "gene_symbol": "DHX29",
  "gene": "UniProtKB:Q7Z478"
}